{
  "gene": "UniProtKB:Q8IWI9",
  "gene_name": "MAX gene-associated protein",
  "term_label": "nucleus",
  "term_id": "GO:0005634",
  "gene_symbol": "MGA"
}